{
  "gene_name": "UDP-GalNAc:beta-1,3-N-acetylgalactosaminyltransferase 1",
  "gene": "UniProtKB:O75752",
  "term_label": "oligosaccharide biosynthetic process",
  "term_id": "GO:0009312",
  "gene_symbol": "B3GALNT1"
}